translational frameshifting [GO:0006452] (biological process) Relationships: is a type of translational elongation [GO:0006414] Regulation: regulated by regulation of translational frameshifting [GO:2001124]; negatively regulated by GO:2001125; positively regulated by positive regulation of translational frameshifting [GO:2001126] Sources: GOC:hjd, ISBN:0195094425 Definition: A mechanism whereby different proteins may result from a single mRNA molecule, due to a change in the parsing of three nucleotides per codon relative to an initiating AUG codon.